{
  "term_id": "GO:0007015",
  "term_label": "actin filament organization",
  "gene": "UniProtKB:P57737",
  "gene_name": "Coronin-7",
  "gene_symbol": "CORO7"
}